mitotic spindle midzone assembly [GO:0051256] (biological process) Also known as: mitotic spindle midzone biogenesis, mitotic spindle midzone biosynthesis, mitotic spindle midzone formation, spindle midzone assembly involved in mitosis, spindle midzone biogenesis involved in mitosis, spindle midzone formation involved in mitosis Definition: The cell cycle process in which the aggregation, arrangement and bonding together of a set of components forms the spindle midzone. References: PMID:24239120 Sources: GOC:mtg_cell_cycle, GOC:vw Relationships: is a type of spindle midzone assembly [GO:0051255]; is a type of GO:1903047; is part of GO:0000022; is part of mitotic spindle assembly [GO:0090307]